{
  "gene": "UniProtKB:P08246",
  "term_label": "acute inflammatory response to antigenic stimulus",
  "gene_name": "Neutrophil elastase",
  "gene_symbol": "ELANE",
  "term_id": "GO:0002438"
}